{
  "gene": "UniProtKB:Q5JVF3",
  "term_id": "GO:0003723",
  "gene_symbol": "PCID2",
  "term_label": "RNA binding",
  "gene_name": "PCI domain-containing protein 2"
}